{
  "gene_symbol": "A0A8V8TPP0",
  "gene_name": "Uncharacterized protein",
  "term_label": "Unknown molecular function",
  "term_id": "UNKNOWN:0001",
  "gene": "UniProtKB:A0A8V8TPP0"
}